{
  "gene_name": "GEM-interacting protein",
  "gene": "UniProtKB:Q9P107",
  "term_label": "intracellular signal transduction",
  "gene_symbol": "GMIP",
  "term_id": "GO:0035556"
}